dihydromonapterin reductase activity [GO:0071172] (molecular function) Relationships: is a type of oxidoreductase activity, acting on the CH-NH group of donors, NAD or NADP as acceptor [GO:0016646] Definition: Catalysis of the reaction: 7,8-dihydromonapterin + NADPH = tetrahydromonapterin + NADP+. References: PMID:19897652 Sources: GOC:imk